{
  "gene_name": "Tubulin polyglutamylase complex subunit 1",
  "gene_symbol": "TPGS1",
  "term_label": "sperm axoneme assembly",
  "term_id": "GO:0007288",
  "gene": "UniProtKB:Q6ZTW0"
}